positive regulation of gastric mucosal blood circulation [GO:1904346] (biological process) Definition: Any process that activates or increases the frequency, rate or extent of gastric mucosal blood circulation. References: PMID:10807413 Sources: GOC:TermGenie, GO_REF:0000058 Relationships: is a type of positive regulation of blood circulation [GO:1903524]; is a type of regulation of gastric mucosal blood circulation [GO:1904344]; positively regulates gastric mucosal blood circulation [GO:1990768] Also known as: positive regulation of stomach mucosal blood circulation, up regulation of gastric mucosal blood circulation, up regulation of stomach mucosal blood circulation, up-regulation of gastric mucosal blood circulation, up-regulation of stomach mucosal blood circulation, upregulation of gastric mucosal blood circulation, upregulation of stomach mucosal blood circulation, activation of gastric mucosal blood circulation, activation of stomach mucosal blood circulation